vascular associated smooth muscle cell differentiation [GO:0035886] (biological process) Subtypes: aortic smooth muscle cell differentiation [GO:0035887], cardiac vascular smooth muscle cell differentiation [GO:0060947], vascular associated smooth muscle cell differentiation involved in phenotypic switching [GO:1905420] Relationships: is a type of smooth muscle cell differentiation [GO:0051145]; is part of GO:0001944 Definition: The process in which a relatively unspecialized cell acquires specialized features of a vascular smooth muscle cell. Also known as: VSMC differentiation, vascular smooth muscle cell differentiation Regulation: regulated by regulation of vascular associated smooth muscle cell differentiation [GO:1905063]; negatively regulated by negative regulation of vascular associated smooth muscle cell differentiation [GO:1905064]; positively regulated by positive regulation of vascular associated smooth muscle cell differentiation [GO:1905065] References: PMID:16151017, PMID:18267954 Sources: GOC:sl